{
  "term_id": "GO:0005737",
  "gene_symbol": "UPF3B",
  "gene": "UniProtKB:Q9BZI7",
  "term_label": "cytoplasm",
  "gene_name": "Regulator of nonsense transcripts 3B"
}